{
  "gene": "UniProtKB:P49841",
  "term_id": "GO:0030424",
  "gene_symbol": "GSK3B",
  "gene_name": "Glycogen synthase kinase-3 beta",
  "term_label": "axon"
}